nuclear migration involved in conjugation with cellular fusion [GO:0000743] (biological process) Also known as: nuclear congression, nuclear migration during conjugation with cellular fusion Relationships: is_a GO:0030473; is part of conjugation with cellular fusion [GO:0000747] References: PMID:16380440 Sources: GOC:clt, GOC:vw Definition: The microtubule-based movement of nuclei towards one another as a prelude to karyogamy in organisms undergoing conjugation with cellular fusion.